transferase activity, transferring alkyl or aryl (other than methyl) groups [GO:0016765] (molecular function) Definition: Catalysis of the transfer of an alkyl or aryl (but not methyl) group from one compound (donor) to another (acceptor). Sources: EC:2.5.1.- Also known as: transferase activity, transferring alkyl or aryl groups, other than methyl groups Relationships: is a type of transferase activity [GO:0016740] Subtypes: 6,7-dimethyl-8-ribityllumazine synthase activity [GO:0000906], GO:0003849, 3-phosphoshikimate 1-carboxyvinyltransferase activity [GO:0003866], O-acetylhomoserine aminocarboxypropyltransferase activity [GO:0003961], cystathionine gamma-synthase activity [GO:0003962], GO:0004124, dihydropteroate synthase activity [GO:0004156], glutathione transferase activity [GO:0004364], GO:0004418, methionine adenosyltransferase activity [GO:0004478], prenyltransferase activity [GO:0004659], GO:0004746, spermidine synthase activity [GO:0004766], thiamine-phosphate diphosphorylase activity [GO:0004789], alkylglycerone-phosphate synthase activity [GO:0008609], 3-deoxy-8-phosphooctulonate synthase activity [GO:0008676], UDP-N-acetylglucosamine 1-carboxyvinyltransferase activity [GO:0008760], corrinoid adenosyltransferase activity [GO:0008817], quinolinate synthetase A activity [GO:0008987], AMP dimethylallyltransferase activity [GO:0009824], thermospermine synthase activity [GO:0010487], tRNA-uridine aminocarboxypropyltransferase activity [GO:0016432], spermine synthase activity [GO:0016768], GO:0030410, GO:0033844, adenosyl-fluoride synthase activity [GO:0033846], O-phosphoserine sulfhydrylase activity [GO:0033847], N2-(2-carboxyethyl)arginine synthase activity [GO:0033848], GO:0033849, Z-farnesyl diphosphate synthase activity [GO:0033850], GO:0033851, deoxyhypusine synthase activity [GO:0034038], GO:0043766, cadaverine aminopropyltransferase activity [GO:0043918], GO:0043919, cysteate synthase activity [GO:0044686], trihydroxypterocarpan dimethylallyltransferase activity [GO:0047292], homospermidine synthase activity [GO:0047296], GO:0047444, beta-pyrazolylalanine synthase activity [GO:0047458], aspulvinone dimethylallyltransferase activity [GO:0047691], discadenine synthase activity [GO:0047870], GO:0050007, sym-norspermidine synthase activity [GO:0050314], thiamine pyridinylase activity [GO:0050332], GO:0050364, zeatin 9-aminocarboxyethyltransferase activity [GO:0050447], GO:0050461, N-acetylneuraminate synthase activity [GO:0050462], uracilylalanine synthase activity [GO:0050471], homospermidine synthase (spermidine-specific) activity [GO:0050514], GO:0052381, ATP/ADP dimethylallyltransferase activity [GO:0052622], GO:0090560, selenomethionine adenosyltransferase activity [GO:0098601], 7,8-dihydropterin-6-yl-methyl-4-(beta-D-ribofuranosyl)aminobenzene 5'-phosphate synthase [GO:0102041], GO:0102522, GO:0102573, 4-hydroxybenzoate geranyltransferase activity [GO:0102930], rRNA small subunit aminocarboxypropyltransferase activity [GO:0106388], 5-amino-6-(D-ribitylamino)uracil--L-tyrosine 4-hydroxyphenyl transferase activity [GO:0141093], cysteine synthase activity, acting on O-succinyl-L-serine [GO:0141223]